{
  "term_id": "UNKNOWN:0002",
  "term_label": "Unknown biological process",
  "gene": "UniProtKB:Q96Q04",
  "gene_name": "Serine_threonine-protein kinase LMTK3",
  "gene_symbol": "LMTK3"
}